{
  "gene_symbol": "WASH2P",
  "term_id": "GO:0055037",
  "term_label": "recycling endosome",
  "gene": "UniProtKB:Q6VEQ5",
  "gene_name": "WAS protein family homolog 2"
}